{
  "term_label": "SCF-dependent proteasomal ubiquitin-dependent protein catabolic process",
  "gene_symbol": "FBXL7",
  "term_id": "GO:0031146",
  "gene_name": "F-box_LRR-repeat protein 7",
  "gene": "UniProtKB:Q9UJT9"
}